locus ceruleus formation [GO:0021705] (biological process) Relationships: is a type of anatomical structure formation involved in morphogenesis [GO:0048646]; is part of pons formation [GO:0021584]; is part of locus ceruleus morphogenesis [GO:0021704] Sources: GOC:cls, GOC:dgh, GOC:dph, GOC:jid, GO_REF:0000021 Definition: The process that gives rise to the locus ceruleus. This process pertains to the initial formation of a structure from unspecified parts. In mice, the locus ceruleus is a dense cluster of neurons within the dorsorostral pons. This nucleus is the major location of neurons that release norepinephrine throughout the brain, and is responsible for physiological responses to stress and panic.